{
  "gene_symbol": "CPXM2",
  "gene_name": "Inactive carboxypeptidase-like protein X2",
  "term_label": "Unknown molecular function",
  "term_id": "UNKNOWN:0001",
  "gene": "UniProtKB:Q8N436"
}